{
  "term_id": "GO:0005737",
  "term_label": "cytoplasm",
  "gene_name": "Tether containing UBX domain for GLUT4",
  "gene_symbol": "ASPSCR1",
  "gene": "UniProtKB:Q9BZE9"
}